regulation of type IV hypersensitivity [GO:0001807] (BP) Definition: Any process that modulates the frequency, rate, or extent of type IV hypersensitivity, a type of inflammatory response. Relationships: is a type of regulation of T cell mediated immunity [GO:0002709]; is a type of regulation of hypersensitivity [GO:0002883]; regulates type IV hypersensitivity [GO:0001806] Sources: GOC:add, ISBN:0781735149 Subtypes: negative regulation of type IV hypersensitivity [GO:0001808], positive regulation of type IV hypersensitivity [GO:0001809]